{
  "gene_symbol": "SNX7",
  "gene": "UniProtKB:Q9UNH6",
  "term_label": "protein transport",
  "gene_name": "Sorting nexin-7",
  "term_id": "GO:0015031"
}